{
  "gene": "UniProtKB:Q7L8W6",
  "term_label": "diphthine-ammonia ligase activity",
  "term_id": "GO:0017178",
  "gene_name": "Diphthine--ammonia ligase",
  "gene_symbol": "DPH6"
}